alkane catabolic process [GO:0043448] (biological process) Also known as: alkane breakdown, alkane catabolism, alkane degradation Relationships: is a type of hydrocarbon catabolic process [GO:0120253] Subtypes: methane catabolic process [GO:0046188] Sources: GOC:jl, Wikipedia:Alkane Definition: The chemical reactions and pathways resulting in the breakdown of an alkane, any acyclic branched or unbranched hydrocarbon having the general formula CnH2n+2.